primary meristem tissue development [GO:0010065] (biological process) Subtypes: ground meristem histogenesis [GO:0010066], GO:0010067, protoderm histogenesis [GO:0010068] Definition: The process whose specific outcome is the progression of the primary meristem over time, from formation to the mature structure, as it occurs during plant embryogenesis. The primary meristem tissue is the protoderm, ground meristem and procambium. Relationships: is a type of embryonic meristem development [GO:0048508] Sources: GOC:tb, ISBN:0471245208 Also known as: primary meristem histogenesis